mitochondrial glutamyl-tRNA aminoacylation [GO:0070149] (biological process) Sources: GOC:mah, GOC:mcc Definition: The process of coupling glutamate to glutamyl-tRNA in a mitochondrion, catalyzed by glutamyl-tRNA synthetase. In tRNA aminoacylation, the amino acid is first activated by linkage to AMP and then transferred to either the 2'- or the 3'-hydroxyl group of the 3'-adenosine residue of the tRNA. Relationships: is a type of GO:0006424; is a type of GO:0070127